{
  "gene": "UniProtKB:P30279",
  "gene_symbol": "CCND2",
  "gene_name": "G1_S-specific cyclin-D2",
  "term_id": "GO:1900087",
  "term_label": "positive regulation of G1/S transition of mitotic cell cycle"
}